{
  "term_label": "transcription coactivator activity",
  "gene_name": "C-terminal-binding protein 2",
  "gene": "UniProtKB:P56545",
  "term_id": "GO:0003713",
  "gene_symbol": "CTBP2"
}